regulation of mesoderm development [GO:2000380] (BP) Subtypes: GO:2000381, positive regulation of mesoderm development [GO:2000382] Sources: GOC:BHF Definition: Any process that modulates the frequency, rate or extent of mesoderm development. Relationships: is a type of regulation of developmental process [GO:0050793]; regulates mesoderm development [GO:0007498]